{
  "term_id": "GO:0032264",
  "gene_name": "Hypoxanthine-guanine phosphoribosyltransferase",
  "gene_symbol": "HPRT1",
  "term_label": "IMP salvage",
  "gene": "UniProtKB:P00492"
}